{
  "gene_name": "Zinc finger protein 556",
  "gene": "UniProtKB:Q9HAH1",
  "term_id": "GO:0000977",
  "term_label": "RNA polymerase II transcription regulatory region sequence-specific DNA binding",
  "gene_symbol": "ZNF556"
}